{
  "gene_symbol": "SOX1",
  "gene_name": "Transcription factor SOX-1",
  "gene": "UniProtKB:O00570",
  "term_id": "GO:0045944",
  "term_label": "positive regulation of transcription by RNA polymerase II"
}